{
  "term_id": "GO:0070166",
  "gene_symbol": "FAM20C",
  "term_label": "enamel mineralization",
  "gene": "UniProtKB:Q8IXL6",
  "gene_name": "Extracellular serine_threonine protein kinase FAM20C"
}